endoplasmic reticulum-Golgi intermediate compartment organization [GO:0097111] (biological process) Definition: A process that is carried out at the cellular level which results in the assembly, arrangement of constituent parts, or disassembly of the endoplasmic reticulum (ER)-Golgi intermediate compartment. Relationships: is a type of organelle organization [GO:0006996] References: PMID:18287528 Sources: GOC:br Also known as: ER-Golgi intermediate compartment organization, ERGIC organization, endoplasmic reticulum-Golgi intermediate compartment organisation, endoplasmic reticulum-Golgi intermediate compartment organization and biogenesis